{
  "gene": "UniProtKB:Q8WZ55",
  "term_id": "GO:0016323",
  "gene_name": "Barttin",
  "term_label": "basolateral plasma membrane",
  "gene_symbol": "BSND"
}